{
  "gene": "UniProtKB:P51606",
  "term_label": "Unknown cellular component",
  "gene_symbol": "RENBP",
  "gene_name": "N-acylglucosamine 2-epimerase",
  "term_id": "UNKNOWN:0003"
}